{
  "gene_symbol": "KRTAP10-9",
  "term_label": "Unknown cellular component",
  "term_id": "UNKNOWN:0003",
  "gene_name": "Keratin-associated protein 10-9",
  "gene": "UniProtKB:P60411"
}